{
  "term_label": "mRNA splicing, via spliceosome",
  "term_id": "GO:0000398",
  "gene": "UniProtKB:Q9Y3C6",
  "gene_symbol": "PPIL1",
  "gene_name": "Peptidyl-prolyl cis-trans isomerase-like 1"
}